{
  "gene_symbol": "ADAM5",
  "gene": "UniProtKB:Q6NVV9",
  "term_id": "UNKNOWN:0003",
  "term_label": "Unknown cellular component",
  "gene_name": "Putative disintegrin and metalloproteinase domain-containing protein 5"
}